protease binding [GO:0002020] (molecular function) Sources: GOC:hjd Relationships: is a type of enzyme binding [GO:0019899] Subtypes: GO:0089720, ubiquitin-specific protease binding [GO:1990381] Definition: Binding to a protease or a peptidase.